{
  "term_id": "GO:0005654",
  "gene": "UniProtKB:Q86Y01",
  "gene_symbol": "DTX1",
  "term_label": "nucleoplasm",
  "gene_name": "E3 ubiquitin-protein ligase DTX1"
}